{
  "gene_symbol": "NFE2L2",
  "term_id": "GO:0006357",
  "gene": "UniProtKB:Q16236",
  "gene_name": "Nuclear factor erythroid 2-related factor 2",
  "term_label": "regulation of transcription by RNA polymerase II"
}